{
  "gene": "UniProtKB:Q15056",
  "gene_name": "Eukaryotic translation initiation factor 4H",
  "gene_symbol": "EIF4H",
  "term_label": "nucleus",
  "term_id": "GO:0005634"
}